{
  "term_id": "GO:0005436",
  "gene_name": "Sodium-dependent phosphate transport protein 2B",
  "gene_symbol": "SLC34A2",
  "gene": "UniProtKB:O95436",
  "term_label": "sodium:phosphate symporter activity"
}